{
  "gene": "UniProtKB:O00270",
  "gene_symbol": "GPR31",
  "gene_name": "12-(S)-hydroxy-5,8,10,14-eicosatetraenoic acid receptor",
  "term_label": "negative regulation of inflammatory response",
  "term_id": "GO:0050728"
}